cardiac neural crest cell delamination [GO:0036036] (biological process) References: PMID:17076275, PMID:18539270, PMID:20490374 Sources: GOC:hjd Subtypes: cardiac neural crest cell delamination involved in outflow tract morphogenesis [GO:1900728] Relationships: is a type of neural crest cell delamination [GO:0036032] Definition: The negative regulation of cell adhesion process in which a cardiac neural crest cell physically separates from the rest of the neural tube.